{
  "term_id": "GO:0005739",
  "term_label": "mitochondrion",
  "gene": "UniProtKB:O60733",
  "gene_name": "85_88 kDa calcium-independent phospholipase A2",
  "gene_symbol": "PLA2G6"
}